{
  "term_id": "GO:0005634",
  "gene": "UniProtKB:Q9ULU4",
  "gene_name": "MYND-type zinc finger-containing chromatin reader ZMYND8",
  "gene_symbol": "ZMYND8",
  "term_label": "nucleus"
}